in_subset [oboInOwl#inSubset]